{
  "term_id": "UNKNOWN:0003",
  "gene_symbol": "ZBTB9",
  "term_label": "Unknown cellular component",
  "gene_name": "Zinc finger and BTB domain-containing protein 9",
  "gene": "UniProtKB:Q96C00"
}